cell projection membrane [GO:0031253] (cellular component) Also known as: membrane extension, membrane projection Sources: GOC:krc, GOC:mah Subtypes: lamellipodium membrane [GO:0031258], GO:0031259, GO:0031260, GO:0031526, filopodium membrane [GO:0031527], microvillus membrane [GO:0031528], ruffle membrane [GO:0032587], neuron projection membrane [GO:0032589], rhabdomere membrane [GO:0033583], muscle cell projection membrane [GO:0036195], GO:0060170, mating projection membrane [GO:0070250], macropinocytic cup membrane [GO:0070686] Definition: The portion of the plasma membrane surrounding a plasma membrane bounded cell surface projection. Relationships: is a type of plasma membrane region [GO:0098590]; is part of plasma membrane bounded cell projection [GO:0120025]